{
  "gene_symbol": "VAT1L",
  "term_id": "UNKNOWN:0002",
  "gene": "UniProtKB:Q9HCJ6",
  "gene_name": "Synaptic vesicle membrane protein VAT-1 homolog-like",
  "term_label": "Unknown biological process"
}